{
  "term_id": "GO:0006955",
  "gene_name": "Immunoglobulin kappa variable 1-9",
  "gene_symbol": "IGKV1-9",
  "term_label": "immune response",
  "gene": "UniProtKB:A0A0C4DH69"
}